{
  "gene_name": "Distal membrane-arm assembly complex protein 2",
  "gene": "UniProtKB:Q9NW81",
  "gene_symbol": "DMAC2",
  "term_label": "mitochondrial respiratory chain complex I assembly",
  "term_id": "GO:0032981"
}